{
  "term_id": "GO:0141014",
  "term_label": "ribosome hibernation",
  "gene": "UniProtKB:A0PJW8",
  "gene_symbol": "DAPL1",
  "gene_name": "Death-associated protein-like 1"
}